{
  "gene_symbol": "PPEF2",
  "gene_name": "Serine_threonine-protein phosphatase with EF-hands 2",
  "term_label": "cytosol",
  "term_id": "GO:0005829",
  "gene": "UniProtKB:O14830"
}